{
  "term_id": "GO:0007283",
  "gene": "UniProtKB:Q15102",
  "gene_symbol": "PAFAH1B3",
  "term_label": "spermatogenesis",
  "gene_name": "Platelet-activating factor acetylhydrolase IB subunit alpha1"
}